{
  "term_id": "GO:0019955",
  "term_label": "cytokine binding",
  "gene_name": "Interleukin-31 receptor subunit alpha",
  "gene_symbol": "IL31RA",
  "gene": "UniProtKB:Q8NI17"
}